{
  "term_label": "neuron differentiation",
  "gene_symbol": "SOX2",
  "gene_name": "Transcription factor SOX-2",
  "gene": "UniProtKB:P48431",
  "term_id": "GO:0030182"
}